endothelial cell activation [GO:0042118] (biological process) Relationships: is a type of GO:0001775 Regulation: regulated by regulation of endothelial cell activation [GO:1904987]; negatively regulated by negative regulation of endothelial cell activation [GO:1904988]; positively regulated by GO:1904989 Subtypes: endothelial cell activation involved in immune response [GO:0002264] Definition: The change in morphology and behavior of an endothelial cell resulting from exposure to a cytokine, chemokine, cellular ligand, or soluble factor. References: PMID:12851652, PMID:14581484 Sources: GOC:mgi_curators, ISBN:0781735149